{
  "term_id": "GO:0005874",
  "gene_name": "Kinesin-like protein KIFC1",
  "gene": "UniProtKB:Q9BW19",
  "gene_symbol": "KIFC1",
  "term_label": "microtubule"
}